mammary gland bud elongation [GO:0060649] (biological process) Definition: The process in which the mammary gland bud grows along its axis. Relationships: is_a developmental growth involved in morphogenesis [GO:0060560]; BFO_0000050 mammary gland bud morphogenesis [GO:0060648] References: PMID:12558599 Sources: GOC:dph